{
  "gene_name": "Nucleoporin NUP35",
  "term_label": "nuclear pore central transport channel",
  "term_id": "GO:0044613",
  "gene": "UniProtKB:Q8NFH5",
  "gene_symbol": "NUP35"
}